mannose-6-phosphate isomerase activity [GO:0004476] (molecular function) Definition: Catalysis of the reaction: D-mannose 6-phosphate = D-fructose 6-phosphate. Relationships: is_a intramolecular oxidoreductase activity, interconverting aldoses and ketoses [GO:0016861] Sources: RHEA:12356 Also known as: phosphohexoisomerase activity, phosphohexomutase activity, D-mannose-6-phosphate aldose-ketose-isomerase activity, D-mannose-6-phosphate ketol-isomerase activity, mannose phosphate isomerase activity, phosphomannoisomerase activity, phosphomannose isomerase activity